retinal blood vessel morphogenesis [GO:0061304] (biological process) Definition: The process whose specific outcome is the progression of a blood vessel of the retina over time, from its formation to the mature structure. Sources: GOC:BHF, GOC:dph Relationships: is a type of blood vessel morphogenesis [GO:0048514]; is a type of retina vasculature morphogenesis in camera-type eye [GO:0061299]